{
  "term_label": "cytoplasm",
  "term_id": "GO:0005737",
  "gene_symbol": "MARCKS",
  "gene_name": "Myristoylated alanine-rich C-kinase substrate",
  "gene": "UniProtKB:P29966"
}